negative regulation of septum digestion after cytokinesis [GO:2001042] (biological process) Sources: GOC:mtg_cell_cycle, GOC:obol Relationships: is a type of regulation of septum digestion after cytokinesis [GO:0010590]; is a type of negative regulation of cellular process [GO:0048523]; negatively regulates GO:0000920 Also known as: negative regulation of cytokinetic cell separation Definition: Any process that stops, prevents or reduces the frequency, rate or extent of the process of physically separating the septal cell wall material by enzymatic digestion, that occurs after daughter cells are separated by cytokinesis.